{
  "term_label": "plasma membrane",
  "gene": "UniProtKB:P21860",
  "gene_name": "Receptor tyrosine-protein kinase erbB-3",
  "gene_symbol": "ERBB3",
  "term_id": "GO:0005886"
}